{
  "gene_symbol": "TMEM121B",
  "gene": "UniProtKB:Q9BXQ6",
  "term_id": "UNKNOWN:0002",
  "term_label": "Unknown biological process",
  "gene_name": "Transmembrane protein 121B"
}